isonocardicin synthase activity [GO:0050007] (molecular function) Relationships: is a type of transferase activity, transferring alkyl or aryl (other than methyl) groups [GO:0016765] Sources: EC:2.5.1.38, RHEA:19845 Also known as: S-adenosyl-L-methionine:nocardicin-E 3-amino-3-carboxypropyltransferase activity, nocardicin aminocarboxypropyltransferase activity Definition: Catalysis of the reaction: S-adenosyl-L-methionine(1+) + nocardicin E = S-methyl-5'-thioadenosine + H+ + isonocardicin A.